{
  "gene": "UniProtKB:P48039",
  "gene_symbol": "MTNR1A",
  "gene_name": "Melatonin receptor type 1A",
  "term_id": "GO:0004930",
  "term_label": "G protein-coupled receptor activity"
}